{
  "term_label": "tRNA modification",
  "gene_name": "Elongator complex protein 5",
  "term_id": "GO:0006400",
  "gene": "UniProtKB:Q8TE02",
  "gene_symbol": "ELP5"
}